endothelin B receptor binding [GO:0031708] (molecular function) Also known as: endothelin B receptor ligand Sources: GOC:mah, GOC:nln Relationships: is a type of GO:0031705 Definition: Binding to an endothelin B receptor.